sphingolipid binding [GO:0046625] (molecular function) Definition: Binding to a sphingolipid, a class of lipids containing the long-chain amine diol sphingosine or a closely related base (a sphingoid). Subtypes: glycosphingolipid binding [GO:0043208], ceramide binding [GO:0097001] Relationships: is a type of GO:0008289 Sources: ISBN:0198506732